{
  "gene": "UniProtKB:A6NM45",
  "gene_name": "Putative claudin-24",
  "term_id": "UNKNOWN:0001",
  "gene_symbol": "CLDN24",
  "term_label": "Unknown molecular function"
}